{
  "gene": "UniProtKB:Q9GZQ4",
  "term_id": "GO:0005886",
  "gene_symbol": "NMUR2",
  "term_label": "plasma membrane",
  "gene_name": "Neuromedin-U receptor 2"
}